{
  "term_label": "DNA-binding transcription factor activity",
  "gene_symbol": "ZNF704",
  "gene_name": "Zinc finger protein 704",
  "term_id": "GO:0003700",
  "gene": "UniProtKB:Q6ZNC4"
}